{
  "gene": "UniProtKB:P15151",
  "term_label": "cell adhesion mediator activity",
  "gene_name": "Poliovirus receptor",
  "gene_symbol": "PVR",
  "term_id": "GO:0098631"
}